positive regulation of sequestering of calcium ion [GO:0051284] (biological process) Sources: GOC:ai Relationships: is a type of positive regulation of cellular process [GO:0048522]; is a type of GO:0051282; positively regulates GO:0051208 Subtypes: negative regulation of release of sequestered calcium ion into cytosol [GO:0051280] Definition: Any process that activates or increases the frequency, rate or extent of the binding or confining calcium ions such that they are separated from other components of a biological system. Also known as: positive regulation of calcium ion (Ca2+) retention, positive regulation of calcium ion (Ca2+) sequestering, positive regulation of calcium ion (Ca2+) sequestration, positive regulation of calcium ion (Ca2+) storage, positive regulation of retention of calcium ion (Ca2+), positive regulation of sequestering of calcium ion (Ca2+), positive regulation of sequestration of calcium ion (Ca2+), positive regulation of storage of calcium ion (Ca2+), up regulation of sequestering of calcium ion, up-regulation of sequestering of calcium ion, upregulation of sequestering of calcium ion, activation of sequestering of calcium ion, stimulation of sequestering of calcium ion